negative regulation of demethylkotanin biosynthetic process [GO:1900653] (biological process) Sources: GOC:TermGenie, GOC:di Also known as: down regulation of demethylkotanin anabolism, down regulation of demethylkotanin biosynthesis, down regulation of demethylkotanin biosynthetic process, down regulation of demethylkotanin formation, down regulation of demethylkotanin synthesis, down-regulation of demethylkotanin anabolism, down-regulation of demethylkotanin biosynthesis, down-regulation of demethylkotanin biosynthetic process, down-regulation of demethylkotanin formation, down-regulation of demethylkotanin synthesis, downregulation of demethylkotanin anabolism, downregulation of demethylkotanin biosynthesis, downregulation of demethylkotanin biosynthetic process, downregulation of demethylkotanin formation, downregulation of demethylkotanin synthesis, inhibition of demethylkotanin anabolism, inhibition of demethylkotanin biosynthesis, inhibition of demethylkotanin formation, inhibition of demethylkotanin synthesis, negative regulation of demethylkotanin anabolism, negative regulation of demethylkotanin biosynthesis, negative regulation of demethylkotanin formation, negative regulation of demethylkotanin synthesis, inhibition of demethylkotanin biosynthetic process Definition: Any process that stops, prevents or reduces the frequency, rate or extent of demethylkotanin biosynthetic process. Relationships: is a type of negative regulation of secondary metabolite biosynthetic process [GO:1900377]; is a type of regulation of demethylkotanin biosynthetic process [GO:1900652]; negatively regulates GO:1900599